linoleic acid metabolic process [GO:0043651] (biological process) Relationships: is a type of GO:0001676; is a type of unsaturated fatty acid metabolic process [GO:0033559]; is a type of olefinic compound metabolic process [GO:0120254] Also known as: linoleic acid metabolism Sources: Wikipedia:Linoleic_Acid Definition: The chemical reactions and pathways involving linoleic acid, an unsaturated omega-6 fatty acid that has the molecular formula C18H32O2.